negative regulation of ATPase-coupled calcium transmembrane transporter activity [GO:1901895] (biological process) Also known as: down regulation of calcium pump, down-regulation of calcium pump, downregulation of calcium pump, inhibition of calcium pump, negative regulation of calcium pump, down regulation of ATP phosphohydrolase (Ca2+-transporting), down regulation of Ca(2+)-transporting ATPase activity, down regulation of Ca2+-pumping ATPase activity, down regulation of Ca2+-transporting ATPase activity, down regulation of calcium transporting ATPase activity, down regulation of calcium-transporting ATPase activity, down-regulation of ATP phosphohydrolase (Ca2+-transporting), down-regulation of Ca(2+)-transporting ATPase activity, down-regulation of Ca2+-pumping ATPase activity, down-regulation of Ca2+-transporting ATPase activity, down-regulation of calcium transporting ATPase activity, down-regulation of calcium-transporting ATPase activity, downregulation of ATP phosphohydrolase (Ca2+-transporting), downregulation of Ca(2+)-transporting ATPase activity, downregulation of Ca2+-pumping ATPase activity, downregulation of Ca2+-transporting ATPase activity, downregulation of calcium transporting ATPase activity, downregulation of calcium-transporting ATPase activity, inhibition of ATP phosphohydrolase (Ca2+-transporting), inhibition of Ca(2+)-transporting ATPase activity, inhibition of Ca2+-pumping ATPase activity, inhibition of Ca2+-transporting ATPase activity, inhibition of calcium transporting ATPase activity, negative regulation of ATP phosphohydrolase (Ca2+-transporting), negative regulation of Ca(2+)-transporting ATPase activity, negative regulation of Ca2+-pumping ATPase activity, negative regulation of Ca2+-transporting ATPase activity, negative regulation of calcium transporting ATPase activity, negative regulation of calcium-transporting ATPase activity, down regulation of calcium ABC transporter, down regulation of calcium efflux ATPase, down regulation of calcium-translocating P-type ATPase activity, down regulation of plasma membrane Ca-ATPase, down regulation of sarco(endo)plasmic reticulum Ca2+-ATPase, down regulation of sarcoplasmic reticulum ATPase, down-regulation of calcium ABC transporter, down-regulation of calcium efflux ATPase, down-regulation of calcium-translocating P-type ATPase activity, down-regulation of plasma membrane Ca-ATPase, down-regulation of sarco(endo)plasmic reticulum Ca2+-ATPase, down-regulation of sarcoplasmic reticulum ATPase, downregulation of calcium ABC transporter, downregulation of calcium efflux ATPase, downregulation of calcium-translocating P-type ATPase activity, downregulation of plasma membrane Ca-ATPase, downregulation of sarco(endo)plasmic reticulum Ca2+-ATPase, downregulation of sarcoplasmic reticulum ATPase, inhibition of calcium ABC transporter, inhibition of calcium efflux ATPase, inhibition of calcium-translocating P-type ATPase activity, inhibition of calcium-transporting ATPase activity, inhibition of plasma membrane Ca-ATPase, inhibition of sarco(endo)plasmic reticulum Ca2+-ATPase, inhibition of sarcoplasmic reticulum ATPase, negative regulation of calcium ABC transporter, negative regulation of calcium efflux ATPase, negative regulation of calcium-translocating P-type ATPase activity, negative regulation of plasma membrane Ca-ATPase, negative regulation of sarco(endo)plasmic reticulum Ca2+-ATPase, negative regulation of sarcoplasmic reticulum ATPase Definition: Any process that stops, prevents or reduces the frequency, rate or extent of an ATPase-coupled calcium transmembrane transporter activity. Relationships: is a type of negative regulation of ATP-dependent activity [GO:0032780]; is a type of negative regulation of calcium ion transmembrane transporter activity [GO:1901020]; is a type of regulation of ATPase-coupled calcium transmembrane transporter activity [GO:1901894]; negatively regulates P-type calcium transporter activity [GO:0005388] References: PMID:19708671 Sources: GOC:BHF, GOC:TermGenie, GOC:rl